penetration of zona pellucida [GO:0007341] (BP) Relationships: is_a GO:0044706; is_a multicellular organismal reproductive process [GO:0048609]; is part of GO:0007338 References: PMID:21755679 Sources: GOC:jl Definition: The infiltration by sperm of the zona pellucida to reach the oocyte. The process involves digestive enzymes from a modified lysosome called the acrosome, situated at the head of the sperm.